{
  "gene": "UniProtKB:Q8WUB2",
  "term_id": "UNKNOWN:0001",
  "term_label": "Unknown molecular function",
  "gene_name": "Protein FAM216A",
  "gene_symbol": "FAM216A"
}